{
  "term_label": "cGMP biosynthetic process",
  "gene_symbol": "NPR2",
  "term_id": "GO:0006182",
  "gene": "UniProtKB:P20594",
  "gene_name": "Atrial natriuretic peptide receptor 2"
}